{
  "term_id": "GO:0005737",
  "gene": "UniProtKB:O43586",
  "term_label": "cytoplasm",
  "gene_name": "Proline-serine-threonine phosphatase-interacting protein 1",
  "gene_symbol": "PSTPIP1"
}